{
  "gene_name": "STING ER exit protein",
  "term_label": "endoplasmic reticulum membrane organization",
  "term_id": "GO:0090158",
  "gene_symbol": "STEEP1",
  "gene": "UniProtKB:Q9H5V9"
}